{
  "term_id": "UNKNOWN:0001",
  "gene": "UniProtKB:Q96KN4",
  "gene_name": "Protein LRATD1",
  "gene_symbol": "LRATD1",
  "term_label": "Unknown molecular function"
}